2-oxoglutarate carboxylase activity [GO:0034029] (molecular function) Definition: Catalysis of the reaction: 2-oxoglutarate + ATP + bicarbonate = ADP + 2 H+ + oxalosuccinate + phosphate. Sources: EC:6.4.1.7, RHEA:20425 Also known as: CFI, OGC, carboxylating factor for ICDH, oxalosuccinate synthetase activity Relationships: is a type of ligase activity, forming carbon-carbon bonds [GO:0016885]